{
  "gene_symbol": "MAN2A2",
  "term_label": "alpha-mannosidase activity",
  "term_id": "GO:0004559",
  "gene": "UniProtKB:P49641",
  "gene_name": "Alpha-mannosidase 2x"
}